{
  "gene_name": "Sodium_hydrogen exchanger 3",
  "term_id": "GO:0051453",
  "gene_symbol": "SLC9A3",
  "term_label": "regulation of intracellular pH",
  "gene": "UniProtKB:P48764"
}